pre-miRNA processing [GO:0031054] (biological process) Regulation: regulated by regulation of pre-miRNA processing [GO:2000631]; negatively regulated by negative regulation of pre-miRNA processing [GO:2000632]; positively regulated by positive regulation of pre-miRNA processing [GO:2000633] References: PMID:15211354 Sources: GOC:sl Also known as: pre-microRNA processing Subtypes: pre-miRNA 3'-end processing [GO:0044747] Definition: A process involved in the conversion of a pre-microRNA transcript into a mature microRNA molecule. Relationships: is a type of miRNA processing [GO:0035196]